{
  "term_label": "Unknown molecular function",
  "gene_name": "T cell receptor alpha joining 21 (Fragment)",
  "gene": "UniProtKB:A0A075B6V2",
  "term_id": "UNKNOWN:0001",
  "gene_symbol": "TRAJ21"
}